{
  "gene_symbol": "PKN1",
  "term_id": "GO:0004674",
  "gene": "UniProtKB:Q16512",
  "term_label": "protein serine/threonine kinase activity",
  "gene_name": "Serine_threonine-protein kinase N1"
}